polymyxin transmembrane transporter activity [GO:0042897] (MF) Also known as: polymyxin transporter activity Relationships: is a type of GO:0042887; is a type of lipid transmembrane transporter activity [GO:0170055]; is part of polymyxin transport [GO:0042893] Definition: Enables the transfer of polymyxin, any of a group of related antibiotics produced by Bacillus polymyxa and active against most Gram-negative bacteria, from one side of a membrane to the other. Sources: GOC:jl, ISBN:0198506732